{
  "gene": "UniProtKB:Q14954",
  "term_id": "GO:0004888",
  "term_label": "transmembrane signaling receptor activity",
  "gene_symbol": "KIR2DS1",
  "gene_name": "Killer cell immunoglobulin-like receptor 2DS1"
}